{
  "gene": "UniProtKB:Q14722",
  "term_label": "juxtaparanode region of axon",
  "gene_name": "Voltage-gated potassium channel subunit beta-1",
  "term_id": "GO:0044224",
  "gene_symbol": "KCNAB1"
}